regulation of polyketide biosynthetic process [GO:1900732] (biological process) Subtypes: regulation of asperfuranone biosynthetic process [GO:1900637], GO:1900670, regulation of F-9775B biosynthetic process [GO:1900675], negative regulation of polyketide biosynthetic process [GO:1900733], positive regulation of polyketide biosynthetic process [GO:1900734], regulation of neosartoricin biosynthetic process [GO:1902053] Definition: Any process that modulates the frequency, rate or extent of polyketide biosynthetic process. Also known as: regulation of polyketide anabolism, regulation of polyketide biosynthesis, regulation of polyketide formation, regulation of polyketide synthesis Sources: GOC:TermGenie, GOC:di Relationships: is a type of regulation of ketone biosynthetic process [GO:0010566]; is a type of regulation of secondary metabolite biosynthetic process [GO:1900376]; RO_0002211 polyketide biosynthetic process [GO:0030639]